{
  "term_id": "GO:0071203",
  "gene_name": "WASH complex subunit 2C",
  "term_label": "WASH complex",
  "gene_symbol": "WASHC2C",
  "gene": "UniProtKB:Q9Y4E1"
}